{
  "gene_name": "Cytoplasmic aconitate hydratase",
  "term_id": "GO:0006879",
  "gene_symbol": "ACO1",
  "gene": "UniProtKB:P21399",
  "term_label": "intracellular iron ion homeostasis"
}